{
  "term_id": "UNKNOWN:0003",
  "gene_symbol": "NANOGNB",
  "term_label": "Unknown cellular component",
  "gene": "UniProtKB:Q7Z5D8",
  "gene_name": "NANOG neighbor homeobox"
}